nuclear cortisol receptor binding [GO:0031961] (molecular function) References: PMID:12511169 Sources: GOC:mah Relationships: is_a nuclear glucocorticoid receptor binding [GO:0035259] Definition: Binding to a nuclear cortisol receptor. Also known as: cortisol receptor binding